positive regulation of response to macrophage colony-stimulating factor [GO:1903971] (biological process) Relationships: is a type of positive regulation of response to cytokine stimulus [GO:0060760]; is a type of regulation of response to macrophage colony-stimulating factor [GO:1903969]; positively regulates response to macrophage colony-stimulating factor [GO:0036005] Also known as: positive regulation of response to M-CSF, positive regulation of response to macrophage colony-stimulating factor stimulus, up regulation of response to M-CSF, up regulation of response to macrophage colony-stimulating factor, up regulation of response to macrophage colony-stimulating factor stimulus, up-regulation of response to M-CSF, up-regulation of response to macrophage colony-stimulating factor, up-regulation of response to macrophage colony-stimulating factor stimulus, upregulation of response to M-CSF, upregulation of response to macrophage colony-stimulating factor, upregulation of response to macrophage colony-stimulating factor stimulus, activation of response to M-CSF, activation of response to macrophage colony-stimulating factor, activation of response to macrophage colony-stimulating factor stimulus Definition: Any process that activates or increases the frequency, rate or extent of response to macrophage colony-stimulating factor. Subtypes: positive regulation of cellular response to macrophage colony-stimulating factor stimulus [GO:1903974] References: PMID:19100238 Sources: GOC:BHF, GOC:TermGenie, GOC:nc, GO_REF:0000058